{
  "term_label": "plasma membrane",
  "gene_symbol": "PIGR",
  "term_id": "GO:0005886",
  "gene_name": "Polymeric immunoglobulin receptor",
  "gene": "UniProtKB:P01833"
}